{
  "term_id": "UNKNOWN:0001",
  "gene": "UniProtKB:Q92837",
  "gene_name": "Proto-oncogene FRAT1",
  "term_label": "Unknown molecular function",
  "gene_symbol": "FRAT1"
}